{
  "term_label": "myosin II complex",
  "gene_name": "Myosin light polypeptide 6",
  "gene": "UniProtKB:P60660",
  "gene_symbol": "MYL6",
  "term_id": "GO:0016460"
}